regulation of development of symbiont in host [GO:0044127] (biological process) Sources: GOC:jl, GOC:pamgo_curators Relationships: is a type of modulation of formation of structure involved in a symbiotic process [GO:0044145]; RO_0002211 development of symbiont in host [GO:0044114] Note: This term partially replaces the obsolete term 'regulation of growth or development of symbiont in host ; GO:0033665'. See also 'regulation of growth of symbiont in host ; GO:0044126'. Subtypes: GO:0044129, negative regulation of development of symbiont in host [GO:0044131] Definition: Any process in which the symbiont regulates its progression from an initial condition to a later condition, within the cells or tissues of the host organism. This may (but not necessarily) include a filamentous growth form, and also can include secretion of proteases and lipases to break down. The host is defined as the larger of the organisms involved in the symbiotic interaction.